{
  "gene_symbol": "NTRK1",
  "term_label": "receptor complex",
  "gene_name": "High affinity nerve growth factor receptor",
  "gene": "UniProtKB:P04629",
  "term_id": "GO:0043235"
}